positive regulation of pentasaccharide transport [GO:1900362] (biological process) Also known as: up regulation of pentasaccharide transport, up-regulation of pentasaccharide transport, upregulation of pentasaccharide transport, activation of pentasaccharide transport Subtypes: positive regulation of maltopentaose transport [GO:1900317] Definition: Any process that activates or increases the frequency, rate or extent of pentasaccharide transport. Sources: GOC:TermGenie, GOC:mengo_curators Relationships: is a type of positive regulation of transport [GO:0051050]; is a type of GO:1900360; positively regulates pentasaccharide transport [GO:2001100]